{
  "gene_symbol": "RBAK",
  "gene": "UniProtKB:Q9NYW8",
  "term_label": "regulation of transcription by RNA polymerase II",
  "term_id": "GO:0006357",
  "gene_name": "RB-associated KRAB zinc finger protein"
}